{
  "gene_name": "Neuralized-like protein 4",
  "gene": "UniProtKB:Q96JN8",
  "gene_symbol": "NEURL4",
  "term_id": "UNKNOWN:0003",
  "term_label": "Unknown cellular component"
}